ATP:phosphate antiporter activity [GO:0140987] (molecular function) Relationships: is a type of ATP transmembrane transporter activity [GO:0005347]; is a type of organophosphate:phosphate antiporter activity [GO:0015315] Also known as: ATP:inorganic phosphate antiporter activity, inorganic phosphate:ATP antiporter activity Definition: Enables the transfer of ATP from one side of a membrane to the other according to the reaction: ATP(out) + phosphate(in) = ATP(in) + phosphate(out). References: PMID:15123600